{
  "gene_name": "Serine_threonine-protein phosphatase PGAM5, mitochondrial",
  "gene_symbol": "PGAM5",
  "term_id": "GO:0004722",
  "term_label": "protein serine/threonine phosphatase activity",
  "gene": "UniProtKB:Q96HS1"
}